{
  "gene_name": "PHD finger protein 20",
  "term_id": "UNKNOWN:0001",
  "term_label": "Unknown molecular function",
  "gene_symbol": "PHF20",
  "gene": "UniProtKB:Q9BVI0"
}